{
  "term_id": "UNKNOWN:0002",
  "gene": "UniProtKB:Q2M243",
  "term_label": "Unknown biological process",
  "gene_name": "Coiled-coil domain-containing protein 27",
  "gene_symbol": "CCDC27"
}